{
  "gene": "UniProtKB:Q9NVN3",
  "term_id": "GO:0005886",
  "term_label": "plasma membrane",
  "gene_name": "Synembryn-B",
  "gene_symbol": "RIC8B"
}